{
  "term_id": "GO:0051897",
  "gene_name": "Rapamycin-insensitive companion of mTOR",
  "gene_symbol": "RICTOR",
  "term_label": "positive regulation of phosphatidylinositol 3-kinase/protein kinase B signal transduction",
  "gene": "UniProtKB:Q6R327"
}